methylaspartate ammonia-lyase activity [GO:0050096] (molecular function) Definition: Catalysis of the reaction: threo-3-methyl-L-aspartate = mesaconate + NH4. Sources: EC:4.3.1.2, RHEA:12829 Relationships: is a type of GO:0016841 Also known as: 3-methylaspartase activity, L-threo-3-methylaspartate ammonia-lyase (mesaconate-forming), L-threo-3-methylaspartate ammonia-lyase activity, beta-methylaspartase activity